{
  "gene_symbol": "TGM2",
  "term_label": "mitochondrion",
  "term_id": "GO:0005739",
  "gene": "UniProtKB:P21980",
  "gene_name": "Protein-glutamine gamma-glutamyltransferase 2"
}